{
  "gene": "UniProtKB:Q8TAE7",
  "term_label": "potassium ion transmembrane transport",
  "gene_name": "Potassium voltage-gated channel subfamily G member 3",
  "gene_symbol": "KCNG3",
  "term_id": "GO:0071805"
}